{
  "term_label": "structural constituent of chromatin",
  "term_id": "GO:0030527",
  "gene": "UniProtKB:Q16695",
  "gene_name": "Histone H3.1t",
  "gene_symbol": "H3-4"
}